response to carbon starvation [GO:0090549] (biological process) References: PMID:18245858 Sources: GOC:tair_curators Relationships: is a type of response to starvation [GO:0042594] Definition: Any process that results in a change in state or activity of a cell or an organism (in terms of movement, secretion, enzyme production, gene expression, etc.) as a result of a starvation stimulus, deprivation of a carbon source.